{
  "gene_name": "Syntaxin-binding protein 6",
  "gene_symbol": "STXBP6",
  "gene": "UniProtKB:Q8NFX7",
  "term_label": "Unknown molecular function",
  "term_id": "UNKNOWN:0001"
}